enucleation [GO:0090601] (biological process) Relationships: is a type of GO:0022411 Definition: The process in which nucleated precursor cells lose their nucleus. Sources: GOC:tb Subtypes: erythrocyte enucleation [GO:0043131], sieve element enucleation [GO:0090602]